{
  "gene_symbol": "THAP8",
  "term_id": "UNKNOWN:0001",
  "gene_name": "THAP domain-containing protein 8",
  "gene": "UniProtKB:Q8NA92",
  "term_label": "Unknown molecular function"
}